detection of wounding [GO:0014822] (biological process) Relationships: is a type of detection of external stimulus [GO:0009581]; is_a GO:0009611 Also known as: detection of injury Definition: The series of events by which an injury stimulus is received and converted into a molecular signal. Sources: GOC:mtg_muscle Subtypes: GO:0014885